{
  "gene_name": "Zinc finger protein 311",
  "term_id": "GO:0000981",
  "gene": "UniProtKB:Q5JNZ3",
  "term_label": "DNA-binding transcription factor activity, RNA polymerase II-specific",
  "gene_symbol": "ZNF311"
}